{
  "gene": "UniProtKB:Q9Y2U8",
  "gene_name": "Inner nuclear membrane protein Man1",
  "gene_symbol": "LEMD3",
  "term_id": "GO:1990446",
  "term_label": "U1 snRNP binding"
}